oxidoreductase activity, acting on paired donors, with incorporation or reduction of molecular oxygen, NAD(P)H as one donor, and incorporation of one atom of oxygen [GO:0016709] (molecular function) Also known as: oxidoreductase activity, acting on paired donors, with incorporation or reduction of molecular oxygen, NADH or NADPH as one donor, and incorporation of one atom of oxygen Subtypes: calcidiol 1-monooxygenase activity [GO:0004498], GO:0004499, GO:0004502, squalene monooxygenase activity [GO:0004506], GO:0004517, GO:0008398, 2-octaprenyl-6-methoxyphenol hydroxylase activity [GO:0008681], 3-(3-hydroxyphenyl)propionate hydroxylase activity [GO:0008688], (+)-abscisic acid 8'-hydroxylase activity [GO:0010295], methane monooxygenase [NAD(P)H] activity [GO:0015049], trans-cinnamate 4-monooxygenase activity [GO:0016710], GO:0016711, vanillate monooxygenase activity [GO:0018489], 4-nitrocatechol 4-monooxygenase activity [GO:0018592], 4-nitrophenol 2-monooxygenase activity [GO:0018601], 4-nitrophenol 4-monooxygenase activity [GO:0018632], dimethyl sulfide monooxygenase activity [GO:0018633], alpha-pinene monooxygenase (NADH) activity [GO:0018634], 1-hydroxy-2-naphthoate hydroxylase activity [GO:0018637], GO:0018638, GO:0018644, alkene monooxygenase activity [GO:0018645], methanesulfonate monooxygenase activity [GO:0018648], toluene-sulfonate methyl-monooxygenase activity [GO:0018652], salicylate 1-monooxygenase activity [GO:0018658], GO:0018659, GO:0018661, phenol 2-monooxygenase activity [GO:0018662], 2,6-dihydroxypyridine 3-monooxygenase activity [GO:0018663], benzoate 4-monooxygenase activity [GO:0018664], 4-hydroxyphenylacetate 1-monooxygenase activity [GO:0018665], 2,4-dichlorophenol 6-monooxygenase activity [GO:0018666], cyclohexanone monooxygenase activity [GO:0018667], 3-hydroxybenzoate 4-monooxygenase activity [GO:0018668], 3-hydroxybenzoate 6-monooxygenase activity [GO:0018669], GO:0018670, 4-hydroxybenzoate 3-monooxygenase [NAD(P)H] activity [GO:0018671], GO:0018672, anthraniloyl-CoA monooxygenase activity [GO:0018673], GO:0018677, 4-hydroxybenzoate 1-hydroxylase activity [GO:0018678], 2-polyprenylphenol 6-hydroxylase activity [GO:0019168], 2-hydroxyquinoline 8-monooxygenase activity [GO:0033766], 4-hydroxyacetophenone monooxygenase activity [GO:0033767], flavonoid 3',5'-hydroxylase activity [GO:0033772], deoxysarpagine hydroxylase activity [GO:0033775], phenylacetone monooxygenase activity [GO:0033776], lithocholate 6beta-hydroxylase activity [GO:0033777], cholesterol 24-hydroxylase activity [GO:0033781], GO:0033784, GO:0034785, trimethylamine monooxygenase activity [GO:0034899], pyrrole-2-carboxylate monooxygenase (NADH) activity [GO:0034938], GO:0036189, cholest-4-en-3-one 26-monooxygenase activity [GO:0036199], ent-isokaurene C2-hydroxylase activity [GO:0036201], ent-cassa-12,15-diene 11-hydroxylase activity [GO:0036202], taxoid 14-beta-hydroxylase activity [GO:0036203], abieta-7,13-dien-18-ol hydroxylase activity [GO:0036204], 9beta-pimara-7,15-diene oxidase activity [GO:0036209], 6-hydroxynicotinate 3-monooxygenase activity [GO:0043731], precorrin-3B synthase activity [GO:0043818], 3,9-dihydroxypterocarpan 6a-monooxygenase activity [GO:0047082], 5-O-(4-coumaroyl)-D-quinate 3'-monooxygenase activity [GO:0047083], methyltetrahydroprotoberberine 14-monooxygenase activity [GO:0047084], hydroxyphenylacetonitrile 2-monooxygenase activity [GO:0047085], ketosteroid monooxygenase activity [GO:0047086], protopine 6-monooxygenase activity [GO:0047087], GO:0047088, dihydrochelirubine 12-monooxygenase activity [GO:0047089], benzoyl-CoA 3-monooxygenase activity [GO:0047090], L-lysine 6-monooxygenase (NADPH) activity [GO:0047091], 4-hydroxyquinoline 3-monooxygenase activity [GO:0047093], 3-hydroxyphenylacetate 6-hydroxylase activity [GO:0047094], 2-hydroxycyclohexanone 2-monooxygenase activity [GO:0047095], GO:0047505, 2-hydroxybiphenyl 3-monooxygenase (NADH) activity [GO:0047544], 2-nitrophenol 2-monooxygenase activity [GO:0047549], GO:0047592, 6-oxocineole dehydrogenase activity [GO:0047597], GO:0047638, anhydrotetracycline monooxygenase activity [GO:0047670], GO:0047717, GO:0047799, GO:0047822, 4'-methoxyisoflavone 2'-hydroxylase activity [GO:0047957], isoflavone 3'-hydroxylase activity [GO:0048000], magnesium-protoporphyrin IX monomethyl ester (oxidative) cyclase activity [GO:0048529], leukotriene-E4 20-monooxygenase activity [GO:0050052], melilotate 3-monooxygenase activity [GO:0050091], GO:0050246, taxifolin 8-monooxygenase activity [GO:0050326], trans-cinnamate 2-monooxygenase activity [GO:0050344], tyrosine N-monooxygenase activity [GO:0050370], quinine 3-monooxygenase activity [GO:0050591], 4-hydroxyphenylacetaldehyde oxime monooxygenase activity [GO:0050592], N-methylcoclaurine 3'-monooxygenase activity [GO:0050593], GO:0050594, vinorine hydroxylase activity [GO:0050596], taxane 10-beta-hydroxylase activity [GO:0050597], GO:0050598, limonene 1,2-monooxygenase [NAD(P)H) activity [GO:0052601], GO:0062186, GO:0072532, tri-(coumaroyl or caffeoyl) spermidine meta-hydroxylase activity [GO:0072533], 4,8,12-trimethyltrideca-1,3,7,11-tetraene synthase activity [GO:0097007], GO:0097008, phenylacetyl-CoA 1,2-epoxidase activity [GO:0097266], isoleucine N-monooxygenase (oxime forming) activity [GO:0102001], valine N-monooxygenase (oxime forming) activity [GO:0102002], 4-nitrotoluene monooxygenase activity [GO:0102037], alpha-humulene 10-hydroxylase activity [GO:0102068], GO:0102099, coniferyl aldehyde 5-hydroxylase activity [GO:0102126], GO:0102134, GO:0102135, GO:0102164, GO:0102169, 5-epi-aristolochene-1,3-dihydroxylase activity [GO:0102170], 4alpha-hydroxymethyl,4beta,14alpha-dimethyl-9beta,19-cyclo-5alpha-ergost-24(241)-en-3beta-ol-4alpha-methyl oxidase activity [GO:0102172], 24-methylenelophenol methyl oxidase activity [GO:0102177], GO:0102180, 1-deoxy-11-oxopentalenate oxygenase activity [GO:0102285], beta-amyrin 11-oxidase activity [GO:0102289], GO:0102320, 2-propylphenol monooxygenase activity [GO:0102322], 2-isopropylphenol monooxygenase activity [GO:0102323], 2,2',3-trihydroxybiphenyl monooxygenase activity [GO:0102325], 11-oxo-beta-amyrin 30-oxidase activity [GO:0102375], GO:0102405, GO:0102464, zeaxanthin 2,2'-beta-hydroxylase activity [GO:0102465], GO:0102517, genkwanin 6-hydroxylase activity [GO:0102532], apigenin-7,4'-dimethyl ether 6-hydroxylase activity [GO:0102534], sakuranetin 6-hydroxylase activity [GO:0102536], dammarenediol 12-hydroxylase activity [GO:0102556], GO:0102557, GO:0102596, GO:0102597, 3alpha-hydroxy-ent-sandaracopimardiene 7-beta-monooxygenase activity [GO:0102598], syn-pimaradiene 6beta-hydroxylase activity [GO:0102612], trimethyluric acid monooxygenase activity [GO:0102613], GO:0102679, L-phenylalanine N-monooxygenase activity [GO:0102684], GO:0102811, GO:0102876, piperitol synthase activity [GO:0102915], GO:0102934, (+)-delta-cadinene-8-hydroxylase activity [GO:0102947], GO:0102995, dimethylsulfoxide oxygenase activity [GO:0103001], 9,10-epoxystearate hydroxylase activity [GO:0103004], 9,10-dihydroxystearate hydroxylase activity [GO:0103006], indole-3-pyruvate monooxygenase activity [GO:0103075], fraxetin 5-hydroxylase activity [GO:0106144], scopoletin 8-hydroxylase activity [GO:0106145], indole-3-carbonyl nitrile 4-hydroxylase activity [GO:0106149], fluorescent chlorophyll catabolite monooxygenase (deformylase) activity [GO:0106371], GO:0120501, 3-demethoxyubiquinone 3-hydroxylase (NADH) activity [GO:0160224] Relationships: is a type of monooxygenase activity [GO:0004497]; is a type of oxidoreductase activity, acting on paired donors, with incorporation or reduction of molecular oxygen [GO:0016705] Sources: EC:1.14.13.- Definition: Catalysis of an oxidation-reduction (redox) reaction in which hydrogen or electrons are transferred from NADH or NADPH and one other donor, and one atom of oxygen is incorporated into one donor.